{
  "gene_name": "Sorting nexin-5",
  "gene": "UniProtKB:Q9Y5X3",
  "gene_symbol": "SNX5",
  "term_label": "dynactin binding",
  "term_id": "GO:0034452"
}